{
  "gene_symbol": "NCR3LG1",
  "term_id": "UNKNOWN:0001",
  "gene": "UniProtKB:Q68D85",
  "gene_name": "Natural cytotoxicity triggering receptor 3 ligand 1",
  "term_label": "Unknown molecular function"
}